{
  "gene": "UniProtKB:Q96S94",
  "term_label": "nucleus",
  "gene_name": "Cyclin-L2",
  "term_id": "GO:0005634",
  "gene_symbol": "CCNL2"
}